{
  "gene_name": "Paralemmin-2",
  "term_id": "UNKNOWN:0003",
  "gene_symbol": "PALM2",
  "gene": "UniProtKB:Q8IXS6",
  "term_label": "Unknown cellular component"
}